{
  "term_label": "signaling receptor activity",
  "gene_name": "Leucine-rich repeats and immunoglobulin-like domains protein 2",
  "gene_symbol": "LRIG2",
  "term_id": "GO:0038023",
  "gene": "UniProtKB:O94898"
}